{
  "gene_symbol": "AUTS2",
  "gene_name": "Autism susceptibility gene 2 protein",
  "term_id": "UNKNOWN:0001",
  "gene": "UniProtKB:Q8WXX7",
  "term_label": "Unknown molecular function"
}